{
  "term_id": "UNKNOWN:0001",
  "gene_name": "Tubulinyl-Tyr carboxypeptidase 1",
  "term_label": "Unknown molecular function",
  "gene": "UniProtKB:Q7L8A9",
  "gene_symbol": "VASH1"
}